{
  "gene_name": "Synapsin-1",
  "gene_symbol": "SYN1",
  "term_label": "synaptic vesicle membrane",
  "term_id": "GO:0030672",
  "gene": "UniProtKB:P17600"
}